viral translational readthrough [GO:0039705] (biological process) Definition: The continuation of translation of a viral mRNA beyond a stop codon by the use of a special tRNA that recognizes the UAG and UGA codons as modified amino acids, rather than as termination codons. References: PMID:10839817 Sources: GOC:bf, GOC:ch, GOC:jl, VZ:859 Note: This term is intended to annotate gene products involved in the process of viral translational readthrough, not viral proteins produced by this translation process. Relationships: is a type of translational readthrough [GO:0006451]; is part of viral translation [GO:0019081] Also known as: viral stop codon readthrough, viral RNA suppression of termination